{
  "gene_name": "Ubiquitin-like-conjugating enzyme ATG3",
  "term_id": "GO:0044804",
  "gene_symbol": "ATG3",
  "term_label": "nucleophagy",
  "gene": "UniProtKB:Q9NT62"
}